{
  "gene_symbol": "SCN2A",
  "gene_name": "Sodium channel protein type 2 subunit alpha",
  "gene": "UniProtKB:Q99250",
  "term_label": "cardiac muscle cell action potential involved in contraction",
  "term_id": "GO:0086002"
}